negative regulation of adenylate cyclase-activating G protein-coupled receptor signaling pathway [GO:0106072] (biological process) Also known as: negative regulation of adenylate cyclase-activating G-protein coupled receptor signaling pathway References: PMID:19246489 Sources: GOC:hjd Subtypes: negative regulation of adenylate cyclase-activating adrenergic receptor signaling pathway [GO:0071878], negative regulation of adenylate cyclase-activating glucose-activated G protein-coupled receptor signaling pathway [GO:0110034] Definition: Any process that stops, prevents or reduces the frequency, rate or extent of an adenylate cyclase-activating G protein-coupled receptor signaling pathway. Relationships: is a type of GO:0045744; is a type of regulation of adenylate cyclase-activating G protein-coupled receptor signaling pathway [GO:0106070]; negatively regulates adenylate cyclase-activating G protein-coupled receptor signaling pathway [GO:0007189]